{
  "gene_name": "WASH complex subunit 2A",
  "gene_symbol": "WASHC2A",
  "term_id": "GO:0071203",
  "gene": "UniProtKB:Q641Q2",
  "term_label": "WASH complex"
}